{
  "gene_symbol": "KIF17",
  "term_label": "cilium",
  "gene_name": "Kinesin-like protein KIF17",
  "gene": "UniProtKB:Q9P2E2",
  "term_id": "GO:0005929"
}